{
  "gene_name": "NEDD4-like E3 ubiquitin-protein ligase WWP2",
  "term_label": "cytoplasm",
  "gene_symbol": "WWP2",
  "term_id": "GO:0005737",
  "gene": "UniProtKB:O00308"
}